poly(3-hydroxyvalerate) biosynthetic process [GO:1902923] (biological process) References: PMID:21705209 Sources: GOC:TermGenie, GOC:mengo_curators, GO_REF:0000068 Also known as: poly(3-hydroxyvalerate) anabolism, poly(3-hydroxyvalerate) biosynthesis, poly(3-hydroxyvalerate) formation, poly(3-hydroxyvalerate) synthesis Relationships: is a type of poly(hydroxyvalerate) biosynthetic process [GO:1902921] Definition: The chemical reactions and pathways resulting in the formation of poly(3-hydroxyvalerate).